negative regulation of action potential [GO:0045759] (biological process) Subtypes: negative regulation of ventricular cardiac muscle cell action potential [GO:1903946], GO:1903948, negative regulation of AV node cell action potential [GO:1903950], negative regulation of neuronal action potential [GO:1904456] Sources: GOC:go_curators Definition: Any process that stops, prevents, or reduces the frequency, rate or extent of action potential creation, propagation or termination. This typically occurs via modulation of the activity or expression of voltage-gated ion channels. Relationships: is a type of negative regulation of biological process [GO:0048519]; is a type of regulation of action potential [GO:0098900]; negatively regulates action potential [GO:0001508] Also known as: down regulation of action potential, down-regulation of action potential, downregulation of action potential, inhibition of action potential